regulation of acylglycerol transport [GO:1901506] (BP) Relationships: is a type of GO:0032368; regulates acylglycerol transport [GO:0034196] Sources: GOC:TermGenie, GOC:sart Subtypes: negative regulation of acylglycerol transport [GO:1901507], positive regulation of acylglycerol transport [GO:1901508], regulation of triglyceride transport [GO:1905883] Also known as: regulation of glyceride transport Definition: Any process that modulates the frequency, rate or extent of acylglycerol transport.